{
  "term_label": "Unknown biological process",
  "gene": "UniProtKB:P0DPF3",
  "gene_name": "Neuroblastoma breakpoint family member 9",
  "term_id": "UNKNOWN:0002",
  "gene_symbol": "NBPF9"
}